{
  "gene_name": "Dual specificity protein phosphatase 18",
  "gene": "UniProtKB:Q8NEJ0",
  "term_label": "cytoplasm",
  "gene_symbol": "DUSP18",
  "term_id": "GO:0005737"
}